{
  "term_label": "Unknown biological process",
  "gene_name": "Nuclear pore complex-interacting protein family member B3",
  "term_id": "UNKNOWN:0002",
  "gene": "UniProtKB:Q92617",
  "gene_symbol": "NPIPB3"
}